{
  "gene_symbol": "KDM1B",
  "term_label": "Unknown biological process",
  "gene_name": "Lysine-specific histone demethylase 2",
  "gene": "UniProtKB:Q8NB78",
  "term_id": "UNKNOWN:0002"
}